{
  "gene_symbol": "IER3",
  "term_id": "GO:0006974",
  "term_label": "DNA damage response",
  "gene_name": "Radiation-inducible immediate-early gene IEX-1",
  "gene": "UniProtKB:P46695"
}